{
  "gene": "UniProtKB:Q9Y2H0",
  "gene_name": "Disks large-associated protein 4",
  "term_label": "glutamatergic synapse",
  "gene_symbol": "DLGAP4",
  "term_id": "GO:0098978"
}